{
  "term_label": "cytosol",
  "term_id": "GO:0005829",
  "gene_symbol": "MOCS2",
  "gene_name": "Molybdopterin synthase catalytic subunit",
  "gene": "UniProtKB:O96007"
}